response to vitamin B2 [GO:0033274] (biological process) Definition: Any process that results in a change in state or activity of a cell or an organism (in terms of movement, secretion, enzyme production, gene expression, etc.) as a result of a vitamin B2 stimulus. Sources: GOC:sl Also known as: response to riboflavin Subtypes: GO:0071302 Relationships: is a type of response to vitamin [GO:0033273]; is a type of response to nitrogen compound [GO:1901698]; is a type of GO:1901700